{
  "term_label": "cytoplasmic vesicle",
  "gene_name": "Guanylate-binding protein 1",
  "gene_symbol": "GBP1",
  "gene": "UniProtKB:P32455",
  "term_id": "GO:0031410"
}